{
  "term_label": "DNA-binding transcription factor activity, RNA polymerase II-specific",
  "term_id": "GO:0000981",
  "gene": "UniProtKB:Q9BXK1",
  "gene_name": "Krueppel-like factor 16",
  "gene_symbol": "KLF16"
}